{
  "gene_symbol": "P2RY13",
  "term_id": "UNKNOWN:0003",
  "term_label": "Unknown cellular component",
  "gene": "UniProtKB:Q9BPV8",
  "gene_name": "P2Y purinoceptor 13"
}